response to ethanol [GO:0045471] (BP) Subtypes: GO:0071361 Regulation: regulated by GO:1901416; RO_0002212 by GO:1901417; positively regulated by positive regulation of response to ethanol [GO:1901418] Definition: Any process that results in a change in state or activity of a cell or an organism (in terms of movement, secretion, enzyme production, gene expression, etc.) as a result of an ethanol stimulus. Relationships: is a type of response to alcohol [GO:0097305] Sources: GOC:go_curators